{
  "gene": "UniProtKB:Q8TF42",
  "gene_symbol": "UBASH3B",
  "term_id": "GO:0051279",
  "gene_name": "Ubiquitin-associated and SH3 domain-containing protein B",
  "term_label": "regulation of release of sequestered calcium ion into cytosol"
}